{
  "term_id": "GO:0005856",
  "gene_name": "Keratin, type I cytoskeletal 15",
  "term_label": "cytoskeleton",
  "gene_symbol": "KRT15",
  "gene": "UniProtKB:P19012"
}